{
  "gene": "UniProtKB:Q9Y2Q1",
  "term_label": "RNA polymerase II cis-regulatory region sequence-specific DNA binding",
  "term_id": "GO:0000978",
  "gene_symbol": "ZNF257",
  "gene_name": "Zinc finger protein 257"
}